{
  "gene_symbol": "PYCARD",
  "term_id": "GO:0002218",
  "term_label": "activation of innate immune response",
  "gene": "UniProtKB:Q9ULZ3",
  "gene_name": "Apoptosis-associated speck-like protein containing a CARD"
}